{
  "gene_symbol": "CACNG5",
  "gene_name": "Voltage-dependent calcium channel gamma-5 subunit",
  "term_id": "GO:0019226",
  "term_label": "transmission of nerve impulse",
  "gene": "UniProtKB:Q9UF02"
}